{
  "gene": "UniProtKB:O14829",
  "gene_name": "Serine_threonine-protein phosphatase with EF-hands 1",
  "term_id": "GO:0005829",
  "term_label": "cytosol",
  "gene_symbol": "PPEF1"
}